{
  "term_label": "single fertilization",
  "gene_name": "Short transient receptor potential channel 3",
  "gene": "UniProtKB:Q13507",
  "term_id": "GO:0007338",
  "gene_symbol": "TRPC3"
}